response to electrical stimulus involved in regulation of muscle adaptation [GO:0014878] (biological process) Definition: Any process that results in a change in state or activity of a cell or an organism (in terms of movement, secretion, enzyme production, gene expression, etc.) as a result of an electrical stimulus. This process occurs as part of the regulation of muscle adaptation. Subtypes: detection of electrical stimulus involved in regulation of muscle adaptation [GO:0014879] Sources: GOC:ef, GOC:mtg_muscle Relationships: is a type of GO:0014874; is a type of response to electrical stimulus [GO:0051602] Also known as: response to electrical stimulus involved in regulation of muscle plasticity